CUA codon-amino acid adaptor activity [GO:0033419] (molecular function) Definition: A triplet codon-amino acid adaptor activity that recognizes a CUA codon. Note: Note that in the standard genetic code, CTA codes for leucine. Relationships: is a type of triplet codon-amino acid adaptor activity [GO:0030533] Also known as: CTA codon-amino acid adaptor activity, leucine tRNA Sources: GOC:mah